{
  "gene": "UniProtKB:O60565",
  "gene_symbol": "GREM1",
  "gene_name": "Gremlin-1",
  "term_label": "extracellular space",
  "term_id": "GO:0005615"
}